{
  "gene_name": "60 kDa heat shock protein, mitochondrial",
  "gene": "UniProtKB:P10809",
  "term_id": "GO:0005759",
  "term_label": "mitochondrial matrix",
  "gene_symbol": "HSPD1"
}